negative regulation of toll-like receptor 15 signaling pathway [GO:2000441] (biological process) Relationships: is a type of negative regulation of immune system process [GO:0002683]; is a type of negative regulation of signal transduction [GO:0009968]; is a type of GO:2000440; negatively regulates toll-like receptor 15 signaling pathway [GO:0035681] Sources: GOC:obol Also known as: negative regulation of TLR15 signaling pathway, negative regulation of toll-like receptor 15 signalling pathway Definition: Any process that stops, prevents or reduces the frequency, rate or extent of toll-like receptor 15 signaling pathway.